{
  "gene": "UniProtKB:Q13595",
  "gene_name": "Transformer-2 protein homolog alpha",
  "term_id": "GO:0005681",
  "gene_symbol": "TRA2A",
  "term_label": "spliceosomal complex"
}